{
  "term_label": "protein maturation",
  "gene": "UniProtKB:Q9BUE6",
  "gene_symbol": "ISCA1",
  "term_id": "GO:0051604",
  "gene_name": "Iron-sulfur cluster assembly 1 homolog, mitochondrial"
}